{
  "gene_name": "FXYD domain-containing ion transport regulator 7",
  "gene_symbol": "FXYD7",
  "term_label": "Unknown cellular component",
  "gene": "UniProtKB:P58549",
  "term_id": "UNKNOWN:0003"
}